{
  "gene": "UniProtKB:Q1L6U9",
  "term_label": "cytoplasm",
  "gene_name": "Prostate-associated microseminoprotein",
  "gene_symbol": "MSMP",
  "term_id": "GO:0005737"
}